{
  "term_id": "GO:0005615",
  "gene_name": "Peptidoglycan recognition protein 4",
  "term_label": "extracellular space",
  "gene_symbol": "PGLYRP4",
  "gene": "UniProtKB:Q96LB8"
}